{
  "gene_symbol": "IGFL3",
  "term_label": "extracellular space",
  "gene": "UniProtKB:Q6UXB1",
  "gene_name": "Insulin growth factor-like family member 3",
  "term_id": "GO:0005615"
}